TFIID-class transcription factor complex binding [GO:0001094] (molecular function) Definition: Binding to a general RNA polymerase II transcription factor belonging to the TFIID complex, one of the factors involved in formation of the preinitiation complex (PIC) by RNA polymerase II. References: PMID:16858867 Sources: GOC:krc Also known as: TFIID-class transcription factor binding Relationships: is_a RNA polymerase II general transcription initiation factor binding [GO:0001091]; is a type of GO:0044877